{
  "term_label": "Unknown cellular component",
  "gene": "UniProtKB:P28290",
  "gene_name": "Protein ITPRID2",
  "gene_symbol": "ITPRID2",
  "term_id": "UNKNOWN:0003"
}